{
  "gene_symbol": "ASCL3",
  "gene_name": "Achaete-scute homolog 3",
  "gene": "UniProtKB:Q9NQ33",
  "term_label": "RNA polymerase II transcription regulator complex",
  "term_id": "GO:0090575"
}